positive regulation of receptor catabolic process [GO:2000646] (biological process) Relationships: is a type of positive regulation of catabolic process [GO:0009896]; is a type of GO:0010604; is a type of regulation of receptor catabolic process [GO:2000644]; positively regulates GO:0032801 Sources: GOC:BHF Also known as: positive regulation of receptor breakdown, positive regulation of receptor catabolism, positive regulation of receptor degradation Definition: Any process that activates or increases the frequency, rate or extent of receptor catabolic process. Subtypes: positive regulation of low-density lipoprotein particle receptor catabolic process [GO:0032805]